{
  "term_label": "Unknown cellular component",
  "gene_name": "Olfactory receptor 9Q1",
  "gene_symbol": "OR9Q1",
  "gene": "UniProtKB:Q8NGQ5",
  "term_id": "UNKNOWN:0003"
}